{
  "term_id": "GO:0047962",
  "term_label": "glycine N-benzoyltransferase activity",
  "gene_name": "Glycine N-acyltransferase",
  "gene_symbol": "GLYAT",
  "gene": "UniProtKB:Q6IB77"
}